{
  "gene": "UniProtKB:A0A0B4J276",
  "gene_name": "T cell receptor alpha variable 25",
  "term_label": "response to bacterium",
  "term_id": "GO:0009617",
  "gene_symbol": "TRAV25"
}